pyruvate fermentation to ethanol [GO:0019655] (biological process) Regulation: RO_0002211 by regulation of glycolytic fermentation to ethanol [GO:2001154]; negatively regulated by GO:2001155; positively regulated by positive regulation of glycolytic fermentation to ethanol [GO:2001172] Sources: GOC:dph, GOC:nr, ISBN:0716720094 Definition: The anaerobic chemical reactions and pathways resulting in the breakdown of pyruvate into ethanol and carbon dioxide (CO2). Also known as: ethanol fermentation, glucose fermentation to ethanol, alcoholic fermentation, ethanol anabolism during fermentation, ethanol biosynthetic process involved in glucose fermentation to ethanol, ethanol formation during fermentation, ethanol synthesis during fermentation, glucose catabolic process to ethanol, glycolytic fermentation to ethanol Relationships: is a type of GO:0006067; is a type of pyruvate fermentation [GO:0019660]